carboxy-cis,cis-muconate cyclase activity [GO:0047768] (molecular function) Sources: EC:5.5.1.5, RHEA:14977 Relationships: is a type of cyclase activity [GO:0009975]; is a type of intramolecular lyase activity [GO:0016872] Definition: Catalysis of the reaction: 3-carboxy-2,5-dihydro-5-oxofuran-2-acetate = 3-carboxy-cis,cis-muconate. Also known as: 3-carboxy-2,5-dihydro-5-oxofuran-2-acetate lyase (decyclizing), 3-carboxy-cis,cis-muconate lactonizing enzyme activity, 3-carboxymuconate cyclase activity